fibroblast growth factor receptor signaling pathway involved in ureteric bud formation [GO:2000699] (BP) Regulation: regulated by GO:2000702; negatively regulated by negative regulation of fibroblast growth factor receptor signaling pathway involved in ureteric bud formation [GO:2000703]; positively regulated by positive regulation of fibroblast growth factor receptor signaling pathway involved in ureteric bud formation [GO:2000704] Sources: GOC:mtg_kidney_jan10, GOC:yaf Definition: The series of molecular signals generated as a consequence of a fibroblast growth factor receptor binding to one of its physiological ligands that contributes to the formation of the ureteric bud from the Wolffian duct. Relationships: is a type of fibroblast growth factor receptor signaling pathway [GO:0008543]; is part of ureteric bud formation [GO:0060676] Also known as: FGF receptor signaling pathway of ureteric bud formation, FGF receptor signalling pathway of ureteric bud formation, FGFR signaling pathway of ureteric bud formation, fibroblast growth factor receptor signaling pathway of ureteric bud formation, fibroblast growth factor receptor signalling pathway of ureteric bud formation